{
  "gene": "UniProtKB:P11912",
  "gene_symbol": "CD79A",
  "term_label": "B cell receptor signaling pathway",
  "term_id": "GO:0050853",
  "gene_name": "B-cell antigen receptor complex-associated protein alpha chain"
}